eclosion rhythm [GO:0008062] (biological process) Definition: The timing of the emergence of the adult fly from its pupal case, which usually occurs at dawn. Relationships: is a type of GO:0048512; is part of eclosion [GO:0007562] References: PMID:11715043